{
  "gene_symbol": "CIAO2B",
  "term_id": "GO:0051604",
  "gene_name": "Cytosolic iron-sulfur assembly component 2B",
  "gene": "UniProtKB:Q9Y3D0",
  "term_label": "protein maturation"
}